{
  "gene_name": "WD repeat domain phosphoinositide-interacting protein 3",
  "gene": "UniProtKB:Q5MNZ6",
  "term_label": "pexophagy",
  "term_id": "GO:0000425",
  "gene_symbol": "WDR45B"
}